{
  "term_label": "single-stranded RNA binding",
  "gene_symbol": "CNBP",
  "gene_name": "CCHC-type zinc finger nucleic acid binding protein",
  "term_id": "GO:0003727",
  "gene": "UniProtKB:P62633"
}